methyltransferase activity [GO:0008168] (molecular function) Definition: Catalysis of the transfer of a methyl group to an acceptor molecule. Sources: ISBN:0198506732 Also known as: methylase Relationships: is_a GO:0016741 Subtypes: C-methyltransferase activity [GO:0008169], N-methyltransferase activity [GO:0008170], GO:0008171, S-methyltransferase activity [GO:0008172], GO:0008173, protein methyltransferase activity [GO:0008276], S-adenosylmethionine-dependent methyltransferase activity [GO:0008757], GO:0009008, GO:0042083, 5-methyltetrahydrofolate-dependent methyltransferase activity [GO:0042084], 5-methyltetrahydropteroyltri-L-glutamate-dependent methyltransferase activity [GO:0042085], 5-methyl-5,6,7,8-tetrahydromethanopterin-dependent methyltransferase activity [GO:0042086], demethylmenaquinone methyltransferase activity [GO:0043770], cobalt-precorrin-6B C5-methyltransferase activity [GO:0043776], cobalt-precorrin-7 C15-methyltransferase activity [GO:0043777], GO:0043780, GO:0043781, cobalt-precorrin-3 C17-methyltransferase activity [GO:0043782], GO:0043791, hydroxyneurosporene-O-methyltransferase activity [GO:0043803], GO:0043819, GO:0043833, trimethylamine methyltransferase activity [GO:0043834], monomethylamine methyltransferase activity [GO:0043852], GO:0044683, methanol-5-hydroxybenzimidazolylcobamide Co-methyltransferase activity [GO:0047152], corydaline synthase activity [GO:0050631], indole acetic acid carboxyl methyltransferase activity [GO:0051749], P-methyltransferase activity [GO:0051994], Se-methyltransferase activity [GO:0051995], selenol Se-methyltransferase activity [GO:0098603], methaneselenol methyltransferase activity [GO:0098613], hydrogen selenide methyltransferase activity [GO:0098614], dimethyl selenide methyltransferase activity [GO:0098615], methyltetrahydrofolate:corrinoid/iron-sulfur protein methyltransferase activity [GO:0102036], demethylrebeccamycin--D-glucose O-methyltransferase activity [GO:0102082], GO:0102109, gibberellin A9 carboxyl methyltransferase activity [GO:0102117], gibberellin A4 carboxyl methyltransferase activity [GO:0102118], malonyl-CoA methyltransferase activity [GO:0102130], tricetin O-methytransferase activity [GO:0102146], 5-methyl-phenazine-1-carboxylate N-methyltransferase activity [GO:0102168], 2-polyprenyl-6-hydroxyphenol methylase activity [GO:0102208], thiocyanate methyltransferase activity [GO:0102215], mycinamicin VI 2''-O-methyltransferase activity [GO:0102302], GO:0102303, GO:0102307, daphnetin-8-O-methyltransferase activity [GO:0102358], quercetin 7-O-methyltransferase activity [GO:0102432], myricetin 7-O-methyltransferase activity [GO:0102435], 3',4',5'-trimethylmyricetin 7-O-methyltransferase activity [GO:0102439], 3',4',5'-trimethylmyricetin 3-O-methyltransferase activity [GO:0102440], GO:0102441, syringetin 3-O-methyltransferase activity [GO:0102442], GO:0102444, 3-methylquercetin 3'-O-methyltransferase activity [GO:0102445], GO:0102446, rhamnetin 3'-O-methyltransferase activity [GO:0102447], rhamnetin 4'-O-methyltransferase activity [GO:0102448], kaempferol 3-O-methyltransferase activity [GO:0102449], kaempferide 7-O-methyltransferase activity [GO:0102450], kaempferide 3-O-methyltransferase activity [GO:0102451], 8-demethylnovobiocic acid C8-methyltransferase activity [GO:0102526], GO:0102529, genkwanin 4'-O-methyltransferase activity [GO:0102533], ladanein 6-O-methyltransferase activity [GO:0102535], GO:0102550, scutellarein 7-methyl ether 6-O-methyltransferase activity [GO:0102623], scutellarein 7-methyl ether 4'-O-methyltransferase activity [GO:0102624], cirsimaritin 4'-O-methyltransferase activity [GO:0102625], 2,7,4'-trihydroxyisoflavanone-4'-O-methyltransferase activity [GO:0102670], 6a-hydroxymaackiain-3-O-methyltransferase activity [GO:0102671], TRIBOA-glucoside methyltransferase activity [GO:0102718], GO:0102741, eriodictyol 3'-O-methyltransferase activity [GO:0102761], eriodictyol 4'-O-methyltransferase activity [GO:0102762], naringenin 7-O-methyltransferase activity [GO:0102766], GO:0102767, GO:0102913, GO:0102917, GO:0102964, 5-n-alk(en)ylresorcinol O-methyltransferase activity [GO:0102990], indole-3-acetate carboxyl methyltransferase activity [GO:0103007], 4-hydroxytryptamine 4-phosphate methyltransferase activity [GO:0140381], GO:0160302, [methyl-Co(III) methanol-specific corrinoid protein]:coenzyme M methyltransferase [GO:1990088] Regulation: positively regulated by tRNA methyltransferase activator activity [GO:0141106]; regulated by methyltransferase regulator activity [GO:0141107]